hydrolase activity, acting on carbon-nitrogen (but not peptide) bonds, in cyclic amidines [GO:0016814] (molecular function) Relationships: is a type of GO:0016810 Definition: Catalysis of the hydrolysis of any non-peptide carbon-nitrogen bond in a cyclic amidine, a compound of the form R-C(=NH)-NH2. Sources: EC:3.5.4.- Subtypes: adenine deaminase activity [GO:0000034], adenosine deaminase activity [GO:0004000], cytidine deaminase activity [GO:0004126], GO:0004131, dCMP deaminase activity [GO:0004132], dihydropterin deaminase activity [GO:0004153], dCTP deaminase activity [GO:0008829], diaminohydroxyphosphoribosylaminopyrimidine deaminase activity [GO:0008835], guanine deaminase activity [GO:0008892], cyclohydrolase activity [GO:0019238], GO:0033973, GO:0034547, N-cyclopropylammeline deaminase activity [GO:0034548], GO:0034549, GO:0035888, 2'-deoxyadenosine deaminase activity [GO:0046936], 1-pyrroline-4-hydroxy-2-carboxylate deaminase activity [GO:0047425], GO:0047623, aminoimidazolase activity [GO:0047664], blasticidin-S deaminase activity [GO:0047711], creatinine deaminase activity [GO:0047790], guanosine deaminase activity [GO:0047974], GO:0050228, pyrithiamine deaminase activity [GO:0050239], S-adenosylhomocysteine deaminase activity [GO:0050270], sepiapterin deaminase activity [GO:0050279], cAMP deaminase activity [GO:0090612], GO:0090613, 5'-methylthioadenosine deaminase activity [GO:0090614], GO:0102127